{
  "term_id": "GO:0005634",
  "term_label": "nucleus",
  "gene_name": "Zinc finger protein 816",
  "gene": "UniProtKB:Q0VGE8",
  "gene_symbol": "ZNF816"
}